{
  "gene": "UniProtKB:O94921",
  "gene_symbol": "CDK14",
  "term_id": "GO:1901987",
  "term_label": "regulation of cell cycle phase transition",
  "gene_name": "Cyclin-dependent kinase 14"
}